positive regulation of leukocyte mediated cytotoxicity [GO:0001912] (biological process) References: PMID:11911826 Sources: GOC:add, ISBN:0781735149 Also known as: positive regulation of immune cell mediated cytotoxicity, positive regulation of leucocyte mediated cytotoxicity, up regulation of leukocyte mediated cytotoxicity, up-regulation of leukocyte mediated cytotoxicity, upregulation of leukocyte mediated cytotoxicity, activation of leukocyte mediated cytotoxicity, stimulation of leukocyte mediated cytotoxicity Relationships: is a type of regulation of leukocyte mediated cytotoxicity [GO:0001910]; is a type of positive regulation of leukocyte mediated immunity [GO:0002705]; is a type of positive regulation of cell killing [GO:0031343]; positively regulates leukocyte mediated cytotoxicity [GO:0001909] Subtypes: positive regulation of antibody-dependent cellular cytotoxicity [GO:0001815], positive regulation of T cell mediated cytotoxicity [GO:0001916], positive regulation of natural killer cell mediated cytotoxicity [GO:0045954], positive regulation of neutrophil mediated cytotoxicity [GO:0070960], positive regulation of microglial cell mediated cytotoxicity [GO:1904151] Definition: Any process that activates or increases the frequency, rate or extent of leukocyte mediated cytotoxicity.